{
  "gene_symbol": "FAM3A",
  "term_id": "GO:0005615",
  "gene": "UniProtKB:P98173",
  "term_label": "extracellular space",
  "gene_name": "Protein FAM3A"
}